{
  "term_id": "GO:0000149",
  "gene": "UniProtKB:Q6PUV4",
  "gene_symbol": "CPLX2",
  "term_label": "SNARE binding",
  "gene_name": "Complexin-2"
}